{
  "gene": "UniProtKB:Q0P5N6",
  "term_id": "UNKNOWN:0001",
  "gene_name": "ADP-ribosylation factor-like protein 16",
  "gene_symbol": "ARL16",
  "term_label": "Unknown molecular function"
}